{
  "term_label": "nucleoplasm",
  "gene_name": "ADP-ribose glycohydrolase MACROD2",
  "term_id": "GO:0005654",
  "gene": "UniProtKB:A1Z1Q3",
  "gene_symbol": "MACROD2"
}